{
  "term_label": "epoxygenase P450 pathway",
  "term_id": "GO:0019373",
  "gene": "UniProtKB:P05181",
  "gene_symbol": "CYP2E1",
  "gene_name": "Cytochrome P450 2E1"
}